Peyer's patch development [GO:0048541] (biological process) Definition: The process whose specific outcome is the progression of Peyer's patches over time, from their formation to the mature structure. Peyer's patches are typically found as nodules associated with gut epithelium with distinct internal structures including B- and T-zones for the activation of lymphocytes. Sources: GOC:add, ISBN:0781735149 Also known as: GALT development, gut-associated lymphoid tissue development Relationships: is a type of mucosa-associated lymphoid tissue development [GO:0048537]